postsynaptic septin cytoskeleton [GO:0150050] (cellular component) References: PMID:28065648 Sources: GOC:aruk, GOC:bc Relationships: is a type of septin cytoskeleton [GO:0032156]; is a type of postsynaptic cytoskeleton [GO:0099571] Definition: The portion of the septin cytoskeleton contained within the postsynapse.